{
  "gene_symbol": "CACNG2",
  "term_label": "AMPA glutamate receptor complex",
  "gene_name": "Voltage-dependent calcium channel gamma-2 subunit",
  "term_id": "GO:0032281",
  "gene": "UniProtKB:Q9Y698"
}